phospholipase C-activating G protein-coupled acetylcholine receptor signaling pathway [GO:0007207] (biological process) Definition: A phospholipase C-activating G protein-coupled receptor signaling pathway initiated by acetylcholine binding to its receptor on the surface of a target cell, and ending with the regulation of a downstream cellular process, e.g. transcription. Sources: GOC:dph, GOC:mah, GOC:signaling, GOC:tb Also known as: activation of phospholipase C activity by muscarinic acetylcholine receptor signalling pathway, muscarinic receptor signaling pathway via activation of PLC, phospholipase C-activating G-protein coupled acetylcholine receptor signaling pathway, activation of phospholipase C activity by G-protein coupled acetylcholine receptor signaling pathway, activation of phospholipase C activity by muscarinic acetylcholine receptor signaling pathway, muscarinic acetylcholine receptor, phospholipase C activating pathway Relationships: is a type of phospholipase C-activating G protein-coupled receptor signaling pathway [GO:0007200]; is a type of GO:0007213